{
  "gene_symbol": "LSM5",
  "gene": "UniProtKB:Q9Y4Y9",
  "gene_name": "U6 snRNA-associated Sm-like protein LSm5",
  "term_id": "GO:0005688",
  "term_label": "U6 snRNP"
}